{
  "term_id": "GO:0031103",
  "gene_symbol": "NREP",
  "gene_name": "Neuronal regeneration-related protein",
  "gene": "UniProtKB:Q16612",
  "term_label": "axon regeneration"
}